{
  "term_label": "Unknown biological process",
  "term_id": "UNKNOWN:0002",
  "gene": "UniProtKB:A6NFN9",
  "gene_name": "Protein ANKUB1",
  "gene_symbol": "ANKUB1"
}